{
  "term_label": "endoplasmic reticulum membrane",
  "gene_symbol": "DERL1",
  "gene_name": "Derlin-1",
  "gene": "UniProtKB:Q9BUN8",
  "term_id": "GO:0005789"
}